nicotinamide metabolic process [GO:0006769] (BP) Definition: The chemical reactions and pathways involving nicotinamide, pyridine-3-carboxamide, the amide of nicotinic acid. It is a member of the B complex of vitamins and occurs widely in living organisms. Also known as: vitamin B3 metabolic process, vitamin B3 metabolism, nicotinamide metabolism, niacin metabolic process, niacin metabolism Subtypes: nicotinamide nucleotide biosynthetic process from niacinamide [GO:0019360] Relationships: is a type of alkaloid metabolic process [GO:0009820]; is a type of amide metabolic process [GO:0043603]; is_a pyridine-containing compound metabolic process [GO:0072524] Sources: ISBN:0198506732